{
  "term_id": "GO:0006357",
  "gene_name": "One cut domain family member 3",
  "gene": "UniProtKB:O60422",
  "term_label": "regulation of transcription by RNA polymerase II",
  "gene_symbol": "ONECUT3"
}